{
  "gene": "UniProtKB:Q6ZMT1",
  "term_label": "Unknown cellular component",
  "gene_name": "SH3 and cysteine-rich domain-containing protein 2",
  "gene_symbol": "STAC2",
  "term_id": "UNKNOWN:0003"
}